{
  "gene_symbol": "CARD8",
  "gene_name": "Caspase recruitment domain-containing protein 8",
  "term_label": "cysteine-type endopeptidase activator activity",
  "term_id": "GO:0140608",
  "gene": "UniProtKB:Q9Y2G2"
}